pyridoxamine transmembrane transport [GO:1903091] (BP) Relationships: is a type of pyridoxamine transport [GO:0031922]; is a type of vitamin transmembrane transport [GO:0035461] References: PMID:15701794 Sources: GOC:TermGenie, GO_REF:0000069 Definition: The process in which pyridoxamine is transported across a membrane.